{
  "term_label": "Unknown cellular component",
  "term_id": "UNKNOWN:0003",
  "gene_name": "Rho-GAP domain-containing protein",
  "gene_symbol": "A0A499FJF3",
  "gene": "UniProtKB:A0A499FJF3"
}